{
  "gene": "UniProtKB:Q0P6D6",
  "gene_symbol": "CCDC15",
  "term_id": "UNKNOWN:0001",
  "gene_name": "Coiled-coil domain-containing protein 15",
  "term_label": "Unknown molecular function"
}